regulation of peptide secretion [GO:0002791] (biological process) Sources: GOC:add Definition: Any process that modulates the frequency, rate, or extent of peptide secretion. Subtypes: negative regulation of peptide secretion [GO:0002792], positive regulation of peptide secretion [GO:0002793], regulation of antimicrobial peptide secretion [GO:0002794], regulation of peptide hormone secretion [GO:0090276] Relationships: is a type of regulation of secretion [GO:0051046]; is a type of regulation of peptide transport [GO:0090087]; RO_0002211 GO:0002790